{
  "gene_name": "Arf-GAP with SH3 domain, ANK repeat and PH domain-containing protein 3",
  "term_label": "ruffle",
  "gene": "UniProtKB:Q8TDY4",
  "term_id": "GO:0001726",
  "gene_symbol": "ASAP3"
}